{
  "gene": "UniProtKB:Q96K78",
  "term_id": "GO:0005886",
  "term_label": "plasma membrane",
  "gene_symbol": "ADGRG7",
  "gene_name": "Adhesion G-protein coupled receptor G7"
}